{
  "term_label": "Unknown molecular function",
  "gene_symbol": "SLC25A35",
  "term_id": "UNKNOWN:0001",
  "gene": "UniProtKB:Q3KQZ1",
  "gene_name": "Solute carrier family 25 member 35"
}